{
  "gene_name": "Acetylcholine receptor subunit gamma",
  "gene": "UniProtKB:P07510",
  "term_id": "GO:0095500",
  "term_label": "acetylcholine receptor signaling pathway",
  "gene_symbol": "CHRNG"
}